metanephric short descending thin limb development [GO:0072271] (biological process) Definition: The process whose specific outcome is the progression of the metanephric short descending thin limb over time, from its formation to the mature structure. The metanephric short descending thin limb is the descending thin limb of a short nephron in the metanephros that has a squamous epithelial morphology. Relationships: is a type of GO:0072063; is a type of GO:0072243; is part of metanephric short nephron development [GO:0072270] Sources: GOC:mtg_kidney_jan10